{
  "term_label": "Wnt receptor catabolic process",
  "term_id": "GO:0038018",
  "gene_symbol": "ZNRF3",
  "gene_name": "E3 ubiquitin-protein ligase ZNRF3",
  "gene": "UniProtKB:Q9ULT6"
}